{
  "gene": "UniProtKB:Q8NBP7",
  "gene_name": "Proprotein convertase subtilisin_kexin type 9",
  "gene_symbol": "PCSK9",
  "term_label": "extracellular space",
  "term_id": "GO:0005615"
}